regulation of cytoplasmic translation [GO:2000765] (biological process) Subtypes: regulation of cytoplasmic translational initiation [GO:1904688], GO:1990497, regulation of cytoplasmic translational termination [GO:1990580], negative regulation of cytoplasmic translation [GO:2000766], positive regulation of cytoplasmic translation [GO:2000767] Relationships: is a type of regulation of translation [GO:0006417]; regulates cytoplasmic translation [GO:0002181] Definition: Any process that modulates the frequency, rate or extent of cytoplasmic translation. Sources: GOC:obol